{
  "gene_symbol": "LRRC66",
  "term_id": "UNKNOWN:0002",
  "term_label": "Unknown biological process",
  "gene_name": "Leucine-rich repeat-containing protein 66",
  "gene": "UniProtKB:Q68CR7"
}